{
  "term_id": "GO:0060048",
  "gene_name": "Telethonin",
  "term_label": "cardiac muscle contraction",
  "gene_symbol": "TCAP",
  "gene": "UniProtKB:O15273"
}